{
  "gene_name": "U3 small nucleolar RNA-associated protein 25 homolog",
  "gene": "UniProtKB:Q68CQ4",
  "gene_symbol": "UTP25",
  "term_id": "GO:0034511",
  "term_label": "U3 snoRNA binding"
}